{
  "term_id": "UNKNOWN:0003",
  "gene": "UniProtKB:O14792",
  "gene_symbol": "HS3ST1",
  "gene_name": "Heparan sulfate glucosamine 3-O-sulfotransferase 1",
  "term_label": "Unknown cellular component"
}